{
  "gene_name": "Prohibitin-2",
  "gene_symbol": "PHB2",
  "term_label": "mitochondrion",
  "gene": "UniProtKB:Q99623",
  "term_id": "GO:0005739"
}